{
  "term_id": "GO:0004890",
  "gene": "UniProtKB:P47870",
  "gene_symbol": "GABRB2",
  "term_label": "GABA-A receptor activity",
  "gene_name": "Gamma-aminobutyric acid receptor subunit beta-2"
}